{
  "term_label": "ERAD pathway",
  "gene_symbol": "USP19",
  "gene_name": "Ubiquitin carboxyl-terminal hydrolase 19",
  "term_id": "GO:0036503",
  "gene": "UniProtKB:O94966"
}